{
  "gene_symbol": "SCYGR8",
  "gene": "UniProtKB:A0A286YFG1",
  "gene_name": "Small cysteine and glycine repeat-containing protein 8",
  "term_id": "UNKNOWN:0003",
  "term_label": "Unknown cellular component"
}